{
  "term_label": "Unknown cellular component",
  "gene": "UniProtKB:Q00765",
  "gene_symbol": "REEP5",
  "term_id": "UNKNOWN:0003",
  "gene_name": "Receptor expression-enhancing protein 5"
}